{
  "gene_symbol": "RHOXF1P3",
  "gene": "UniProtKB:A0A994J3T1",
  "term_label": "Unknown cellular component",
  "term_id": "UNKNOWN:0003",
  "gene_name": "Rhox homeobox family member 1 pseudogene 3"
}